{
  "gene_symbol": "POLR2E",
  "gene_name": "DNA-directed RNA polymerases I, II, and III subunit RPABC1",
  "term_label": "RNA polymerase III complex",
  "term_id": "GO:0005666",
  "gene": "UniProtKB:P19388"
}